{
  "gene": "UniProtKB:Q3LI70",
  "term_label": "Unknown molecular function",
  "term_id": "UNKNOWN:0001",
  "gene_name": "Keratin-associated protein 19-6",
  "gene_symbol": "KRTAP19-6"
}